skeletal muscle satellite stem cell maintenance involved in skeletal muscle regeneration [GO:0098731] (biological process) Definition: Any process by which the number of skeletal muscle satellite stem cells in a skeletal muscle is maintained during skeletal muscle regeneration. There are at least two mechanisms by which this is achieved. Skeletal muscle satellite stem cell asymmetric division ensures satellite stem cell numbers are kept constant. Symmetric division of these cells amplifies the number of skeletal muscle satellite stem cells. References: PMID:23303905 Relationships: is a type of skeletal muscle satellite cell maintenance involved in skeletal muscle regeneration [GO:0014834]; is a type of somatic stem cell population maintenance [GO:0035019]